{
  "gene_name": "Paired box protein Pax-4",
  "gene_symbol": "PAX4",
  "gene": "UniProtKB:O43316",
  "term_id": "UNKNOWN:0003",
  "term_label": "Unknown cellular component"
}